{
  "gene_name": "Hepatoma-derived growth factor",
  "term_id": "UNKNOWN:0001",
  "gene_symbol": "HDGF",
  "term_label": "Unknown molecular function",
  "gene": "UniProtKB:P51858"
}